IMP biosynthetic process [GO:0006188] (biological process) Also known as: IMP anabolism, IMP biosynthesis, IMP formation, IMP synthesis Relationships: is a type of purine ribonucleotide biosynthetic process [GO:0009152]; is a type of GO:0009168; is a type of GO:0046040 Sources: ISBN:0198506732 Definition: The chemical reactions and pathways resulting in the formation of IMP, inosine monophosphate. Subtypes: 'de novo' IMP biosynthetic process [GO:0006189], GO:0032264